{
  "term_label": "actin cytoskeleton",
  "term_id": "GO:0015629",
  "gene_name": "Protein PEAK3",
  "gene": "UniProtKB:Q6ZS72",
  "gene_symbol": "PEAK3"
}